{
  "gene": "UniProtKB:Q5SV97",
  "gene_name": "PGC-1 and ERR-induced regulator in muscle protein 1",
  "term_label": "cytoplasm",
  "gene_symbol": "PERM1",
  "term_id": "GO:0005737"
}